regulation of interleukin-26 production [GO:0032670] (biological process) Definition: Any process that modulates the frequency, rate, or extent of interleukin-26 production. Also known as: regulation of IL-26 production, regulation of interleukin-26 biosynthetic process Relationships: is a type of regulation of cytokine production [GO:0001817]; regulates interleukin-26 production [GO:0032630] Subtypes: negative regulation of interleukin-26 production [GO:0032710], positive regulation of interleukin-26 production [GO:0032750] Sources: GOC:mah